modulation of zoospore encystment on host [GO:0075219] (BP) Subtypes: positive regulation of zoospore encystment on host [GO:0075220], negative regulation of zoospore encystment on host [GO:0075221] Sources: GOC:pamgo_curators Definition: Any process that modulates the frequency, rate or extent of zoospore encystment on host. The host is defined as the larger of the organisms involved in a symbiotic interaction. Relationships: is a type of modulation of spore encystment on host [GO:0075215]; regulates zoospore encystment on host [GO:0075218]